actin modification [GO:0030047] (biological process) Relationships: is a type of actin cytoskeleton organization [GO:0030036]; is a type of protein modification process [GO:0036211] Definition: Covalent modification of an actin molecule. Sources: GOC:mah Subtypes: actin ubiquitination [GO:0007014]